{
  "gene_name": "Olfactory receptor 10A4",
  "gene_symbol": "OR10A4",
  "term_label": "plasma membrane",
  "term_id": "GO:0005886",
  "gene": "UniProtKB:Q9H209"
}